{
  "term_id": "GO:0005737",
  "gene_name": "Exportin-4",
  "gene": "UniProtKB:Q9C0E2",
  "term_label": "cytoplasm",
  "gene_symbol": "XPO4"
}